{
  "term_label": "RNA polymerase II transcription regulatory region sequence-specific DNA binding",
  "gene_name": "Zinc finger BED domain-containing protein 2",
  "term_id": "GO:0000977",
  "gene": "UniProtKB:Q9BTP6",
  "gene_symbol": "ZBED2"
}